{
  "gene_name": "Amelogenin, X isoform",
  "term_id": "GO:0030345",
  "gene": "UniProtKB:Q99217",
  "gene_symbol": "AMELX",
  "term_label": "structural constituent of tooth enamel"
}